ligand-gated channel activity [GO:0022834] (molecular function) Sources: GOC:mtg_transport, ISBN:0815340729 Relationships: is a type of gated channel activity [GO:0022836] Definition: Enables the transmembrane transfer of a solute by a channel that opens when a specific ligand has been bound by the channel complex or one of its constituent parts. Subtypes: ligand-gated monoatomic ion channel activity [GO:0015276], transmitter-gated channel activity [GO:0022835], monoatomic ion-gated channel activity [GO:0022839], ATP-gated ion channel activity [GO:0035381], intracellularly calcium-gated channel activity [GO:0141147]